xylan binding [GO:2001062] (molecular function) Definition: Binding to xylan. Relationships: is a type of polysaccharide binding [GO:0030247] Sources: GOC:mengo_curators Subtypes: arabinoxylan binding [GO:2001068]